{
  "gene_name": "Sulfite oxidase, mitochondrial",
  "term_id": "GO:0005739",
  "gene_symbol": "SUOX",
  "gene": "UniProtKB:P51687",
  "term_label": "mitochondrion"
}